{
  "gene_symbol": "ZZEF1",
  "term_id": "UNKNOWN:0003",
  "gene_name": "Zinc finger ZZ-type and EF-hand domain-containing protein 1",
  "term_label": "Unknown cellular component",
  "gene": "UniProtKB:O43149"
}